{
  "gene": "UniProtKB:Q16594",
  "term_id": "GO:0000124",
  "gene_name": "Transcription initiation factor TFIID subunit 9",
  "term_label": "SAGA complex",
  "gene_symbol": "TAF9"
}